positive regulation of developmental process [GO:0051094] (biological process) Sources: GOC:ai Subtypes: GO:0002636, positive regulation of mitochondrial fusion [GO:0010636], GO:0031496, positive regulation of mammary gland epithelial cell proliferation [GO:0033601], positive regulation of embryonic development [GO:0040019], positive regulation of vulval development [GO:0040026], positive regulation of sporulation [GO:0043938], positive regulation of cell differentiation [GO:0045597], GO:0045684, positive regulation of salivary gland boundary specification [GO:0045706], positive regulation of chitin-based cuticle tanning [GO:0045801], positive regulation of isotype switching [GO:0045830], positive regulation of retinal cell programmed cell death [GO:0046670], positive regulation of cuticle pigmentation [GO:0048081], GO:0048091, positive regulation of male pigmentation [GO:0048093], positive regulation of post-embryonic development [GO:0048582], GO:0048636, GO:0048639, positive regulation of hair follicle development [GO:0051798], positive regulation of nervous system development [GO:0051962], positive regulation of syncytium formation by plasma membrane fusion [GO:0060143], positive regulation of mammary placode formation by mesenchymal-epithelial signaling [GO:0060617], positive regulation of epithelial cell proliferation involved in prostate gland development [GO:0060769], positive regulation of floral organ abscission [GO:0060861], positive regulation of dendritic spine development [GO:0060999], positive regulation of cartilage development [GO:0061036], GO:0061169, positive regulation of sclerotome development [GO:0061189], positive regulation of entry into reproductive diapause [GO:0061965], positive regulation of somatic muscle development [GO:0062224], positive regulation of biomineral tissue development [GO:0070169], GO:0070572, positive regulation of germ tube formation [GO:0075011], positive regulation of appressorium formation [GO:0075018], positive regulation of formation of symbiont germ tube hook structure for appressorium development [GO:0075031], positive regulation of penetration peg formation [GO:0075055], GO:0075185, positive regulation of hyphopodium formation [GO:0075189], positive regulation of haustorium mother cell formation [GO:0075194], positive regulation of symbiont haustorium neck formation for entry into host [GO:0075199], positive regulation of penetration hypha formation [GO:0075203], positive regulation of spore-bearing organ development [GO:0075261], positive regulation of synapse maturation [GO:0090129], positive regulation of mitochondrial fission [GO:0090141], positive regulation of kidney development [GO:0090184], GO:0110013, GO:0110039, positive regulation of placenta blood vessel development [GO:0110080], positive regulation of animal organ morphogenesis [GO:0110110], GO:0110138, positive regulation of neuron projection arborization [GO:0150012], positive regulation of dendrite development [GO:1900006], positive regulation of leaf senescence [GO:1900057], positive regulation of bone trabecula formation [GO:1900156], GO:1901165, positive regulation of cardiac chamber morphogenesis [GO:1901221], GO:1901492, positive regulation of muscle tissue development [GO:1901863], positive regulation of sclerotium development [GO:1901924], positive regulation of seed dormancy process [GO:1902040], positive regulation of shoot apical meristem development [GO:1902185], positive regulation of stem cell population maintenance [GO:1902459], GO:1902764, GO:1902865, positive regulation of retina development in camera-type eye [GO:1902868], GO:1902917, GO:1903012, positive regulation of lactation [GO:1903489], positive regulation of vasculature development [GO:1904018], positive regulation of adipose tissue development [GO:1904179], GO:1904250, GO:1904261, positive regulation of spore germination [GO:1904361], positive regulation of cardiac ventricle development [GO:1904414], positive regulation of thyroid gland epithelial cell proliferation [GO:1904443], GO:1904655, GO:1904747, GO:1905142, positive regulation of vascular associated smooth muscle cell dedifferentiation [GO:1905176], positive regulation of cardiac myofibril assembly [GO:1905306], positive regulation of morphogenesis of an epithelium [GO:1905332], positive regulation of plant organ morphogenesis [GO:1905423], positive regulation of branching morphogenesis of a nerve [GO:1905492], GO:1905623, positive regulation of artery morphogenesis [GO:1905653], positive regulation of dauer entry [GO:1905911], positive regulation of cell fate determination [GO:1905935], positive regulation of gonad development [GO:1905941], GO:2000017, positive regulation of mammary stem cell proliferation [GO:2000103], positive regulation of myotome development [GO:2000287], positive regulation of fibroblast growth factor receptor signaling pathway involved in neural plate anterior/posterior pattern formation [GO:2000315], GO:2000334, positive regulation of mesoderm development [GO:2000382], GO:2000385, positive regulation of ovarian follicle development [GO:2000386], positive regulation of lamellipodium morphogenesis [GO:2000394], positive regulation of optic nerve formation [GO:2000597], positive regulation of seed maturation [GO:2000693], positive regulation of mesenchymal cell proliferation involved in ureter development [GO:2000729], positive regulation of anterior head development [GO:2000744], GO:2000792, positive regulation of metanephric ureteric bud development [GO:2001076] Also known as: up regulation of developmental process, up-regulation of developmental process, upregulation of developmental process, activation of developmental process, stimulation of developmental process Definition: Any process that activates or increases the rate or extent of development, the biological process whose specific outcome is the progression of an organism over time from an initial condition (e.g. a zygote, or a young adult) to a later condition (e.g. a multicellular animal or an aged adult). Relationships: is a type of GO:0048518; is a type of GO:0050793; positively regulates GO:0032502